{
  "gene_name": "Glutamate-rich protein 6B",
  "gene_symbol": "ERICH6B",
  "gene": "UniProtKB:Q5W0A0",
  "term_id": "UNKNOWN:0001",
  "term_label": "Unknown molecular function"
}